passive transmembrane transporter activity [GO:0022803] (molecular function) Also known as: porters, uniporter activity z, facilitated diffusion Subtypes: channel activity [GO:0015267] Sources: GOC:mtg_transport, ISBN:0815340729 Relationships: is a type of GO:0022857 Definition: Enables the transfer of a single solute from one side of a membrane to the other by a mechanism involving conformational change, either by facilitated diffusion or in a membrane potential dependent process if the solute is charged.